{
  "gene": "UniProtKB:Q7Z2H8",
  "term_id": "GO:0005774",
  "gene_symbol": "SLC36A1",
  "gene_name": "Proton-coupled amino acid transporter 1",
  "term_label": "vacuolar membrane"
}